{
  "term_label": "Unknown cellular component",
  "gene": "UniProtKB:P59020",
  "gene_name": "Down syndrome critical region protein 9",
  "term_id": "UNKNOWN:0003",
  "gene_symbol": "DSCR9"
}